floral whorl structural organization [GO:0048459] (biological process) Sources: GOC:PO_curators, GOC:jid, PO:0025023 Definition: The process that contributes to the act of creating the structural organization of the floral whorl. This process pertains to the physical shaping of a rudimentary structure. Relationships: is a type of developmental process involved in reproduction [GO:0003006]; is a type of anatomical structure arrangement [GO:0048532]; is part of floral whorl morphogenesis [GO:0048457]; is part of flower structural organization [GO:0048461] Also known as: floral whorl structural organisation